mesangial cell-matrix adhesion [GO:0035759] (biological process) Definition: The binding of a mesangial cell to the extracellular matrix via adhesion molecules. A mesangial cell is a cell that encapsulates the capillaries and venules in the kidney. References: PMID:15569314 Sources: CL:0000650, GOC:BHF Relationships: is_a cell-matrix adhesion [GO:0007160]